{
  "gene": "UniProtKB:O14810",
  "term_label": "synaptic vesicle exocytosis",
  "gene_symbol": "CPLX1",
  "term_id": "GO:0016079",
  "gene_name": "Complexin-1"
}